{
  "term_label": "positive regulation of autophagy",
  "gene_name": "GATOR complex protein NPRL3",
  "term_id": "GO:0010508",
  "gene": "UniProtKB:Q12980",
  "gene_symbol": "NPRL3"
}